{
  "gene": "UniProtKB:Q9UL16",
  "gene_name": "Cilia- and flagella-associated protein 45",
  "term_label": "Unknown cellular component",
  "gene_symbol": "CFAP45",
  "term_id": "UNKNOWN:0003"
}